{
  "term_label": "ribosomal large subunit biogenesis",
  "term_id": "GO:0042273",
  "gene_name": "Large ribosomal subunit protein eL33",
  "gene": "UniProtKB:P18077",
  "gene_symbol": "RPL35A"
}